{
  "gene": "UniProtKB:P15924",
  "term_id": "GO:0098609",
  "gene_symbol": "DSP",
  "gene_name": "Desmoplakin",
  "term_label": "cell-cell adhesion"
}